{
  "term_label": "nucleus",
  "term_id": "GO:0005634",
  "gene_name": "Zinc finger protein 652",
  "gene": "UniProtKB:Q9Y2D9",
  "gene_symbol": "ZNF652"
}